NAD+-protein-lysine ADP-ribosyltransferase activity [GO:0140804] (molecular function) Relationships: is_a NAD+-protein mono-ADP-ribosyltransferase activity [GO:1990404] References: PMID:25043379 Sources: RHEA:58220 Definition: Catalysis of the reaction: L-lysyl-[protein] + NAD+ = H+ + N(6)-(ADP-D-ribosyl)-L-lysyl-[protein] + nicotinamide.